{
  "gene_name": "Electrogenic aspartate_glutamate antiporter SLC25A12, mitochondrial",
  "term_id": "GO:0015810",
  "gene_symbol": "SLC25A12",
  "term_label": "aspartate transmembrane transport",
  "gene": "UniProtKB:O75746"
}